{
  "gene": "UniProtKB:Q9Y305",
  "term_label": "mitochondrion",
  "gene_symbol": "ACOT9",
  "gene_name": "Acyl-coenzyme A thioesterase 9, mitochondrial",
  "term_id": "GO:0005739"
}